{
  "term_label": "synapse",
  "term_id": "GO:0045202",
  "gene_symbol": "CHRNB2",
  "gene_name": "Neuronal acetylcholine receptor subunit beta-2",
  "gene": "UniProtKB:P17787"
}